{
  "term_id": "GO:0034431",
  "gene_symbol": "NUDT4B",
  "gene_name": "Diphosphoinositol polyphosphate phosphohydrolase NUDT4B",
  "gene": "UniProtKB:A0A024RBG1",
  "term_label": "bis(5'-adenosyl)-hexaphosphatase activity"
}